{
  "term_id": "UNKNOWN:0003",
  "gene_symbol": "MINPP1",
  "term_label": "Unknown cellular component",
  "gene_name": "Multiple inositol polyphosphate phosphatase 1",
  "gene": "UniProtKB:Q9UNW1"
}